{
  "gene_symbol": "CMPK2",
  "term_id": "GO:0004550",
  "term_label": "nucleoside diphosphate kinase activity",
  "gene_name": "UMP-CMP kinase 2, mitochondrial",
  "gene": "UniProtKB:Q5EBM0"
}